{
  "gene": "UniProtKB:P55061",
  "term_id": "GO:0005262",
  "term_label": "calcium channel activity",
  "gene_symbol": "TMBIM6",
  "gene_name": "Bax inhibitor 1"
}